{
  "gene_name": "Nuclear transcription factor Y subunit beta",
  "term_label": "CCAAT-binding factor complex",
  "gene_symbol": "NFYB",
  "term_id": "GO:0016602",
  "gene": "UniProtKB:P25208"
}